{
  "gene_name": "Zinc finger protein PLAGL2",
  "term_label": "nucleus",
  "term_id": "GO:0005634",
  "gene_symbol": "PLAGL2",
  "gene": "UniProtKB:Q9UPG8"
}